substrate-dependent cell migration [GO:0006929] (biological process) Also known as: substrate-bound cell migration Definition: The orderly movement of a cell from one site to another along a substrate such as the extracellular matrix; the migrating cell forms a protrusion that attaches to the substrate. References: PMID:11944043, PMID:14657486 Sources: ISBN:0815316194 Relationships: is a type of GO:0016477 Subtypes: GO:0021825, extracellular matrix-dependent thymocyte migration [GO:0072680]